{
  "gene_name": "Zinc finger protein 492",
  "gene": "UniProtKB:Q9P255",
  "term_id": "GO:0006355",
  "term_label": "regulation of DNA-templated transcription",
  "gene_symbol": "ZNF492"
}